{
  "term_id": "GO:0002503",
  "gene": "UniProtKB:P13765",
  "gene_symbol": "HLA-DOB",
  "gene_name": "HLA class II histocompatibility antigen, DO beta chain",
  "term_label": "peptide antigen assembly with MHC class II protein complex"
}